{
  "term_label": "nucleolus",
  "term_id": "GO:0005730",
  "gene": "UniProtKB:Q9H7B2",
  "gene_name": "Ribosome production factor 2 homolog",
  "gene_symbol": "RPF2"
}